{
  "term_label": "Unknown cellular component",
  "gene": "UniProtKB:Q06250",
  "gene_name": "Putative Wilms tumor upstream neighbor 1 gene protein",
  "term_id": "UNKNOWN:0003",
  "gene_symbol": "WT1-AS"
}